negative regulation of imaginal disc-derived wing vein specification [GO:0110109] (biological process) References: PMID:11861482 Sources: GOC:ha Definition: Any process that stops, prevents, or reduces the frequency, rate or extent of imaginal disc-derived wing vein specification. Relationships: is_a negative regulation of multicellular organismal process [GO:0051241]; is a type of regulation of imaginal disc-derived wing vein specification [GO:0110107]; negatively regulates imaginal disc-derived wing vein specification [GO:0007474]